{
  "term_label": "carbohydrate binding",
  "term_id": "GO:0030246",
  "gene": "UniProtKB:P08236",
  "gene_symbol": "GUSB",
  "gene_name": "Beta-glucuronidase"
}